{
  "gene_name": "LHFPL tetraspan subfamily member 4 protein",
  "gene": "UniProtKB:Q7Z7J7",
  "gene_symbol": "LHFPL4",
  "term_id": "GO:0097112",
  "term_label": "gamma-aminobutyric acid receptor clustering"
}